ABC-type oligosaccharide transporter activity [GO:0015422] (molecular function) Definition: Enables the transfer of a solute or solutes from one side of a membrane to the other according to the reaction: ATP + H2O + oligosaccharide(out) = ADP + phosphate + oligosaccharide(in). Sources: EC:7.5.2.2 Also known as: oligosaccharide ABC transporter, ABC-type oligosaccharide transporter, ATP-dependent oligosaccharide transmembrane transporter activity, ATPase-coupled oligosaccharide transmembrane transporter activity, oligosaccharide-transporting ATPase activity Relationships: is a type of oligosaccharide transmembrane transporter activity [GO:0015157]; is_a ABC-type carbohydrate transporter activity [GO:0043211] Subtypes: GO:0015423, ABC-type oligogalacturonide transporter activity [GO:0033154]